{
  "gene_name": "Proto-oncogene Wnt-3",
  "gene_symbol": "WNT3",
  "term_label": "frizzled binding",
  "gene": "UniProtKB:P56703",
  "term_id": "GO:0005109"
}